{
  "gene": "UniProtKB:Q9H156",
  "gene_name": "SLIT and NTRK-like protein 2",
  "gene_symbol": "SLITRK2",
  "term_id": "GO:0051965",
  "term_label": "positive regulation of synapse assembly"
}